T=3 icosahedral viral capsid [GO:0039617] (cellular component) Relationships: is a type of icosahedral viral capsid [GO:0019030] Sources: VZ:806 Definition: The protein coat that surrounds the infective nucleic acid in some virus particles where the subunits (capsomeres) are arranged to form an icosahedron with T=3 symmetry. The T=3 capsid is composed of 12 pentameric and 20 hexameric capsomeres.